{
  "term_id": "GO:0032281",
  "gene_name": "Brorin",
  "gene": "UniProtKB:Q2TAL6",
  "gene_symbol": "VWC2",
  "term_label": "AMPA glutamate receptor complex"
}